{
  "term_label": "Unknown biological process",
  "gene": "UniProtKB:E9PQX1",
  "gene_name": "Cation channel sperm-associated auxiliary subunit TMEM262",
  "term_id": "UNKNOWN:0002",
  "gene_symbol": "TMEM262"
}